{
  "gene_name": "DENN domain-containing protein 10",
  "gene_symbol": "DENND10",
  "gene": "UniProtKB:Q8TCE6",
  "term_id": "GO:0031267",
  "term_label": "small GTPase binding"
}